{
  "term_id": "GO:0015187",
  "gene_symbol": "SLC32A1",
  "gene_name": "Vesicular inhibitory amino acid transporter",
  "gene": "UniProtKB:Q9H598",
  "term_label": "glycine transmembrane transporter activity"
}